{
  "term_id": "GO:0006361",
  "gene_symbol": "RRN3",
  "gene_name": "RNA polymerase I-specific transcription initiation factor RRN3",
  "gene": "UniProtKB:Q9NYV6",
  "term_label": "transcription initiation at RNA polymerase I promoter"
}